N',N'',N'''-triacetylfusarinine C biosynthetic process [GO:1900551] (biological process) Relationships: is a type of GO:0044550 Regulation: RO_0002211 by regulation of N',N'',N'''-triacetylfusarinine C biosynthetic process [GO:1900695]; negatively regulated by GO:1900696; positively regulated by positive regulation of N',N'',N'''-triacetylfusarinine C biosynthetic process [GO:1900697] Sources: GOC:TermGenie, GOC:di Definition: The chemical reactions and pathways resulting in the formation of N',N'',N'''-triacetylfusarinine C. Also known as: N',N'',N'''-triacetylfusarinine C anabolism, N',N'',N'''-triacetylfusarinine C biosynthesis, N',N'',N'''-triacetylfusarinine C formation, N',N'',N'''-triacetylfusarinine C synthesis